siRNA-mediated gene silencing by mRNA destabilization [GO:0090625] (biological process) Relationships: is a type of mRNA destabilization [GO:0061157]; is a type of siRNA-mediated post-transcriptional gene silencing [GO:0140766] Subtypes: siRNA-mediated long-distance post-transcriptional gene silencing [GO:0010495] Definition: An siRNA-mediated post-transcriptional gene silencing pathway in which small interfering RNAs (siRNAs) direct the cleavage of target mRNAs. Once incorporated into a RNA-induced silencing complex (RISC), an siRNA will typically direct cleavage by base pairing with perfect or near-perfect complementarity to the target mRNA. References: PMID:15260970 Sources: GOC:BHF, GOC:BHF_miRNA, GOC:rph Also known as: gene silencing by mRNA cleavage, mRNA cleavage involved in gene silencing by siRNA, mRNA destabilization-mediated gene silencing by siRNA